{
  "gene_symbol": "SLC40A1",
  "term_id": "GO:0005381",
  "term_label": "iron ion transmembrane transporter activity",
  "gene_name": "Solute carrier family 40 member 1",
  "gene": "UniProtKB:Q9NP59"
}